{
  "gene_symbol": "ZNF354B",
  "term_id": "GO:0000978",
  "gene": "UniProtKB:Q96LW1",
  "gene_name": "Zinc finger protein 354B",
  "term_label": "RNA polymerase II cis-regulatory region sequence-specific DNA binding"
}